{
  "gene_name": "Gamma-crystallin S",
  "term_id": "GO:0002088",
  "gene_symbol": "CRYGS",
  "term_label": "lens development in camera-type eye",
  "gene": "UniProtKB:P22914"
}